retinal cell apoptotic process [GO:1990009] (BP) Definition: Any apoptotic process in a retinal cell. References: PMID:15558487, PMID:24664675 Sources: GOC:mtg_apoptosis Relationships: is a type of apoptotic process [GO:0006915] Also known as: induction of retinal programmed cell death Subtypes: retinal rod cell apoptotic process [GO:0097473], retinal cone cell apoptotic process [GO:0097474], compound eye retinal cell apoptotic process [GO:1990010]